{
  "gene_name": "1,4-alpha-glucan-branching enzyme",
  "gene_symbol": "GBE1",
  "gene": "UniProtKB:Q04446",
  "term_label": "glycogen biosynthetic process",
  "term_id": "GO:0005978"
}